positive regulation of endothelin production [GO:1904472] (biological process) Definition: Any process that activates or increases the frequency, rate or extent of endothelin production. References: PMID:15560120 Sources: GOC:TermGenie, GO_REF:0000058 Also known as: up regulation of endothelin secretion, up-regulation of endothelin secretion, upregulation of endothelin secretion, activation of EDN1 secretion, activation of EDN2 secretion, activation of EDN3 secretion, activation of endothelin secretion, activation of endothelin-1 secretion, activation of endothelin-2 secretion, activation of endothelin-3 secretion, positive regulation of EDN1 secretion, positive regulation of EDN2 secretion, positive regulation of EDN3 secretion, positive regulation of endothelin secretion, positive regulation of endothelin-1 secretion, positive regulation of endothelin-2 secretion, positive regulation of endothelin-3 secretion, up regulation of EDN1 secretion, up regulation of EDN2 secretion, up regulation of EDN3 secretion, up regulation of endothelin-1 secretion, up regulation of endothelin-2 secretion, up regulation of endothelin-3 secretion, up-regulation of EDN1 secretion, up-regulation of EDN2 secretion, up-regulation of EDN3 secretion, up-regulation of endothelin-1 secretion, up-regulation of endothelin-2 secretion, up-regulation of endothelin-3 secretion, upregulation of EDN1 secretion, upregulation of EDN2 secretion, upregulation of EDN3 secretion, upregulation of endothelin-1 secretion, upregulation of endothelin-2 secretion, upregulation of endothelin-3 secretion Relationships: is a type of positive regulation of cytokine production [GO:0001819]; is a type of regulation of endothelin production [GO:1904470]; positively regulates GO:1990775